{
  "gene_symbol": "DHX9",
  "term_label": "positive regulation of transcription by RNA polymerase II",
  "term_id": "GO:0045944",
  "gene_name": "ATP-dependent RNA helicase A",
  "gene": "UniProtKB:Q08211"
}